phlobaphene biosynthetic process [GO:0051559] (biological process) Definition: The chemical reactions and pathways resulting in the formation of phlobaphenes, red pigments with oligomeric or polymeric structure derived from the flavonoid intermediate flavan-4-ols. Relationships: is a type of biosynthetic process [GO:0009058]; is a type of pigment biosynthetic process [GO:0046148] References: PMID:11402179